{
  "gene_symbol": "CYTH4",
  "gene_name": "Cytohesin-4",
  "gene": "UniProtKB:Q9UIA0",
  "term_id": "GO:0016192",
  "term_label": "vesicle-mediated transport"
}